phosphatidylinositol 3-kinase complex, class II [GO:0097652] (cellular component) Relationships: is a type of phosphatidylinositol 3-kinase complex [GO:0005942] References: PMID:24587488 Sources: GOC:ha Also known as: class II PI3K complex, class II phosphatidylinositol 3-kinase complex Definition: A phosphatidylinositol 3-kinase complex that contains a catalytic subunit of a phosphatidylinositol 3-kinase (PI3K) enzyme and one or more adaptor proteins. There is no known obligatory regulatory subunit. The class II PI3K (PI3KC2) subfamily of genes has members in vertebrates, worm and fly, but none in yeast.